{
  "term_id": "UNKNOWN:0001",
  "gene_name": "RAD9, HUS1, RAD1-interacting nuclear orphan protein 1",
  "term_label": "Unknown molecular function",
  "gene_symbol": "RHNO1",
  "gene": "UniProtKB:Q9BSD3"
}